beta-1,2-oligomannoside metabolic process [GO:0070135] (biological process) References: PMID:18234669 Sources: GOC:mah Relationships: is a type of mannan metabolic process [GO:0010412] Subtypes: GO:0070136 Also known as: beta-1,2-oligomannoside metabolism Definition: The chemical reactions and pathways involving beta-1,2-linked oligomannosides, which are found in fungal cell wall phosphopeptidomannan and phospholipomannan.